{
  "gene_name": "Metalloreductase STEAP1",
  "term_id": "GO:0005768",
  "gene": "UniProtKB:Q9UHE8",
  "gene_symbol": "STEAP1",
  "term_label": "endosome"
}